{
  "gene": "UniProtKB:P26232",
  "term_id": "GO:0016477",
  "gene_name": "Catenin alpha-2",
  "gene_symbol": "CTNNA2",
  "term_label": "cell migration"
}